{
  "gene_symbol": "KCNIP1",
  "gene_name": "Kv channel-interacting protein 1",
  "term_id": "GO:0008076",
  "gene": "UniProtKB:Q9NZI2",
  "term_label": "voltage-gated potassium channel complex"
}